{
  "gene_name": "High affinity immunoglobulin gamma Fc receptor I",
  "gene_symbol": "FCGR1A",
  "term_label": "IgG binding",
  "gene": "UniProtKB:P12314",
  "term_id": "GO:0019864"
}